{
  "gene_name": "Cytotoxic and regulatory T-cell molecule",
  "gene": "UniProtKB:O95727",
  "gene_symbol": "CRTAM",
  "term_label": "plasma membrane",
  "term_id": "GO:0005886"
}